{
  "term_label": "Unknown cellular component",
  "gene": "UniProtKB:Q8TF64",
  "term_id": "UNKNOWN:0003",
  "gene_symbol": "GIPC3",
  "gene_name": "PDZ domain-containing protein GIPC3"
}